{
  "gene_name": "P antigen family member 2",
  "gene_symbol": "PAGE2",
  "gene": "UniProtKB:Q7Z2X7",
  "term_label": "Unknown biological process",
  "term_id": "UNKNOWN:0002"
}